{
  "term_label": "endomembrane system",
  "term_id": "GO:0012505",
  "gene_name": "Membrane-associated progesterone receptor component 2",
  "gene": "UniProtKB:O15173",
  "gene_symbol": "PGRMC2"
}